pronephric proximal tubule development [GO:0035776] (biological process) References: PMID:18787069 Sources: GOC:mtg_kidney_jan10, GOC:yaf Relationships: is a type of pronephric nephron tubule development [GO:0039020]; is a type of proximal tubule development [GO:0072014] Definition: The progression of the pronephric proximal tubule over time, from its formation to the mature structure. A pronephric nephron tubule is an epithelial tube that is part of the pronephros.